{
  "term_label": "Unknown biological process",
  "term_id": "UNKNOWN:0002",
  "gene_symbol": "NDUFB7",
  "gene": "UniProtKB:P17568",
  "gene_name": "NADH dehydrogenase [ubiquinone] 1 beta subcomplex subunit 7"
}